{
  "term_id": "GO:0005634",
  "gene_symbol": "JAZF1",
  "gene": "UniProtKB:Q86VZ6",
  "term_label": "nucleus",
  "gene_name": "Juxtaposed with another zinc finger protein 1"
}